{
  "term_id": "GO:0000981",
  "term_label": "DNA-binding transcription factor activity, RNA polymerase II-specific",
  "gene_name": "Transcription factor SOX-10",
  "gene": "UniProtKB:P56693",
  "gene_symbol": "SOX10"
}